positive regulation of nucleotide catabolic process [GO:0030813] (biological process) Sources: GOC:mah Definition: Any process that activates or increases the frequency, rate or extent of the chemical reactions and pathways resulting in the breakdown of nucleotides. Relationships: is_a positive regulation of catabolic process [GO:0009896]; is_a regulation of nucleotide catabolic process [GO:0030811]; is a type of GO:0045981; positively regulates nucleotide catabolic process [GO:0009166] Subtypes: positive regulation of purine nucleotide catabolic process [GO:0033123] Also known as: positive regulation of nucleotide breakdown, positive regulation of nucleotide catabolism, positive regulation of nucleotide degradation, up regulation of nucleotide catabolic process, up-regulation of nucleotide catabolic process, upregulation of nucleotide catabolic process, activation of nucleotide catabolic process, stimulation of nucleotide catabolic process